{
  "gene_symbol": "ZMYND15",
  "gene_name": "Zinc finger MYND domain-containing protein 15",
  "term_label": "Unknown cellular component",
  "term_id": "UNKNOWN:0003",
  "gene": "UniProtKB:Q9H091"
}